{
  "gene": "UniProtKB:Q9UN76",
  "term_id": "GO:0001762",
  "gene_name": "Sodium- and chloride-dependent neutral and basic amino acid transporter B(0+)",
  "gene_symbol": "SLC6A14",
  "term_label": "beta-alanine transport"
}